regulation of response to stimulus [GO:0048583] (biological process) Relationships: is a type of regulation of biological process [GO:0050789]; regulates response to stimulus [GO:0050896] Note: Note that this term is in the subset of terms that should not be used for direct gene product annotation. Instead, select a child term or, if no appropriate child term exists, please request a new term. Direct annotations to this term may be amended during annotation QC. Sources: GOC:jid Subtypes: regulation of response to biotic stimulus [GO:0002831], GO:0009966, regulation of response to external stimulus [GO:0032101], GO:0032107, regulation of muscle adaptation [GO:0043502], GO:0045304, positive regulation of response to stimulus [GO:0048584], negative regulation of response to stimulus [GO:0048585], regulation of immune response [GO:0050776], regulation of response to cytokine stimulus [GO:0060759], regulation of response to stress [GO:0080134], regulation of cellular response to growth factor stimulus [GO:0090287], regulation of olfactory learning [GO:0090328], regulation of thermomorphogenesis [GO:0140920], GO:1900067, regulation of cellular response to insulin stimulus [GO:1900076], regulation of filamentous growth of a population of unicellular organisms in response to chemical stimulus [GO:1900437], regulation of response to pullulan [GO:1900518], regulation of response to amylopectin [GO:1900521], regulation of filamentous growth of a population of unicellular organisms in response to pH [GO:1900741], regulation of response to alcohol [GO:1901419], regulation of response to cycloalkane [GO:1901431], regulation of response to furfural [GO:1901442], regulation of response to benzene [GO:1901451], regulation of response to toluene [GO:1901454], regulation of response to acetate [GO:1901457], regulation of response to formic acid [GO:1901460], regulation of cellular response to manganese ion [GO:1905802], regulation of cellular response to oxidopamine [GO:1905846], GO:1905890, regulation of response to calcium ion [GO:1905945], regulation of photoperiodism, flowering [GO:2000028], regulation of response to red or far red light [GO:2000030], regulation of cellular response to testosterone stimulus [GO:2000654], regulation of cellular response to X-ray [GO:2000683], regulation of detection of glucose [GO:2000970], GO:2001023, regulation of response to gamma radiation [GO:2001228] Definition: Any process that modulates the frequency, rate or extent of a response to a stimulus. Response to stimulus is a change in state or activity of a cell or an organism (in terms of movement, secretion, enzyme production, gene expression, etc.) as a result of a stimulus.